cerebroside-sulfatase activity [GO:0004098] (molecular function) Relationships: is a type of sulfuric ester hydrolase activity [GO:0008484] Also known as: cerebroside-sulphatase activity, arylsulfatase A activity, cerebroside sulfate sulfatase activity, cerebroside-3-sulfate 3-sulfohydrolase activity Definition: Catalysis of the reaction: a cerebroside 3-sulfate + H2O = a cerebroside + sulfate. Sources: EC:3.1.6.8